{
  "gene": "UniProtKB:P35548",
  "term_id": "GO:0048598",
  "gene_symbol": "MSX2",
  "term_label": "embryonic morphogenesis",
  "gene_name": "Homeobox protein MSX-2"
}